{
  "gene_name": "Plastin-3",
  "term_label": "actin filament binding",
  "gene": "UniProtKB:P13797",
  "gene_symbol": "PLS3",
  "term_id": "GO:0051015"
}